regulation of secondary growth [GO:2000603] (BP) Relationships: is a type of regulation of growth [GO:0040008]; regulates secondary growth [GO:0080117] Sources: GOC:obol Subtypes: negative regulation of secondary growth [GO:2000604], positive regulation of secondary growth [GO:2000605] Definition: Any process that modulates the frequency, rate or extent of secondary growth.